regulation of imaginal disc growth [GO:0045570] (biological process) Relationships: is a type of regulation of developmental growth [GO:0048638]; regulates GO:0007446 Definition: Any process that modulates the frequency, rate or extent of the growth of the imaginal disc. Subtypes: negative regulation of imaginal disc growth [GO:0045571], positive regulation of imaginal disc growth [GO:0045572] Sources: GOC:go_curators